negative regulation of basement membrane assembly involved in embryonic body morphogenesis [GO:1904260] (biological process) Relationships: is a type of GO:0051093; is_a negative regulation of extracellular matrix assembly [GO:1901202]; is a type of regulation of basement membrane assembly involved in embryonic body morphogenesis [GO:1904259]; negatively regulates basement membrane assembly involved in embryonic body morphogenesis [GO:2001197] Definition: Any process that stops, prevents or reduces the frequency, rate or extent of basement membrane assembly involved in embryonic body morphogenesis. Also known as: down regulation of basement membrane assembly involved in embryonic body morphogenesis, down-regulation of basement membrane assembly involved in embryonic body morphogenesis, downregulation of basement membrane assembly involved in embryonic body morphogenesis, inhibition of basement membrane assembly involved in embryonic body morphogenesis References: PMID:23940118 Sources: GOC:TermGenie, GOC:als, GO_REF:0000058